kidney vasculature morphogenesis [GO:0061439] (biological process) Subtypes: glomerulus vasculature morphogenesis [GO:0072103] Definition: The process in which the kidney vasculature is generated and organized. Morphogenesis pertains to the creation of form. Sources: GOC:dph, GOC:mtg_kidney_jan10 Relationships: is a type of anatomical structure morphogenesis [GO:0009653]; is part of renal system vasculature morphogenesis [GO:0061438]; is part of kidney vasculature development [GO:0061440]